{
  "gene_symbol": "HOXA7",
  "term_id": "GO:0000978",
  "gene": "UniProtKB:P31268",
  "term_label": "RNA polymerase II cis-regulatory region sequence-specific DNA binding",
  "gene_name": "Homeobox protein Hox-A7"
}